{
  "gene_symbol": "CASS4",
  "gene_name": "Cas scaffolding protein family member 4",
  "term_id": "GO:0007169",
  "term_label": "cell surface receptor protein tyrosine kinase signaling pathway",
  "gene": "UniProtKB:Q9NQ75"
}